{
  "gene": "UniProtKB:Q9HB65",
  "gene_symbol": "ELL3",
  "term_id": "GO:0000987",
  "gene_name": "RNA polymerase II elongation factor ELL3",
  "term_label": "cis-regulatory region sequence-specific DNA binding"
}